{
  "gene_name": "Succinate dehydrogenase assembly factor 4, mitochondrial",
  "term_label": "mitochondrion",
  "term_id": "GO:0005739",
  "gene_symbol": "SDHAF4",
  "gene": "UniProtKB:Q5VUM1"
}